R8 cell differentiation [GO:0045465] (BP) Regulation: regulated by regulation of R8 cell differentiation [GO:0045679]; negatively regulated by GO:0045680; RO_0002213 by positive regulation of R8 cell differentiation [GO:0045681] References: PMID:11880339 Relationships: is a type of compound eye photoreceptor cell differentiation [GO:0001751] Definition: The process in which a relatively unspecialized cell acquires the specialized features of the R8 photoreceptor.